{
  "term_id": "UNKNOWN:0002",
  "term_label": "Unknown biological process",
  "gene_name": "Migration and invasion-inhibitory protein",
  "gene_symbol": "MIIP",
  "gene": "UniProtKB:Q5JXC2"
}